{
  "gene": "UniProtKB:Q99469",
  "gene_name": "SH3 and cysteine-rich domain-containing protein",
  "gene_symbol": "STAC",
  "term_label": "skeletal muscle contraction",
  "term_id": "GO:0003009"
}